{
  "gene": "UniProtKB:A6NFK2",
  "term_id": "GO:0005902",
  "gene_symbol": "GRXCR2",
  "term_label": "microvillus",
  "gene_name": "Glutaredoxin domain-containing cysteine-rich protein 2"
}